{
  "term_label": "transmembrane transporter activity",
  "gene_name": "Choline transporter-like protein 5",
  "term_id": "GO:0022857",
  "gene_symbol": "SLC44A5",
  "gene": "UniProtKB:Q8NCS7"
}